lipopolysaccharide 3-alpha-galactosyltransferase activity [GO:0008918] (molecular function) Sources: EC:2.4.1.44, GOC:mr Also known as: LPS 3-alpha-galactosyltransferase activity, lipopolysaccharide galactosyltransferase activity, lipopolysaccharide-alpha-1,3-D-galactosyltransferase, UDP-galactose:lipopolysaccharide 3-alpha-D-galactosyltransferase activity, UDP-galactose:lipopolysaccharide alpha,3-galactosyltransferase activity, UDP-galactose:polysaccharide galactosyltransferase activity, UDPgalactose:lipopolysaccharide 3-alpha-D-galactosyltransferase activity, lipopolysaccharide 1,3-galactosyltransferase activity, uridine diphosphate galactose:lipopolysaccharide alpha-3-galactosyltransferase activity, uridine diphosphogalactose-lipopolysaccharide alpha,3-galactosyltransferase activity Relationships: is a type of UDP-galactosyltransferase activity [GO:0035250]; is part of lipopolysaccharide biosynthetic process [GO:0009103] Definition: Catalysis of the reaction: UDP-galactose + lipopolysaccharide = UDP + 1,3 alpha-D-galactosyl-lipopolysaccharide.